{
  "gene_symbol": "SNAPC3",
  "gene": "UniProtKB:Q92966",
  "gene_name": "snRNA-activating protein complex subunit 3",
  "term_label": "RNA polymerase II cis-regulatory region sequence-specific DNA binding",
  "term_id": "GO:0000978"
}